{
  "gene": "UniProtKB:Q96EA4",
  "term_id": "GO:0000132",
  "gene_symbol": "SPDL1",
  "gene_name": "Protein Spindly",
  "term_label": "establishment of mitotic spindle orientation"
}